{
  "term_id": "GO:0016592",
  "gene_symbol": "MED7",
  "gene_name": "Mediator of RNA polymerase II transcription subunit 7",
  "term_label": "mediator complex",
  "gene": "UniProtKB:O43513"
}